{
  "term_id": "GO:0004252",
  "gene_symbol": "TPSAB1",
  "gene": "UniProtKB:Q15661",
  "term_label": "serine-type endopeptidase activity",
  "gene_name": "Tryptase alpha_beta-1"
}